outer dense plaque of desmosome [GO:0090636] (cellular component) Definition: The desmosomal part containing plakoglobins, plakophilins, the N-termini of desmoplakins, as well as the cytoplasmic tails of the desmosomal cadherins, which together attach the plaque to the plasma membrane. References: PMID:20066089 Relationships: is a type of cellular anatomical structure [GO:0110165]; BFO_0000050 GO:0030057